female pronucleus [GO:0001939] (cellular component) Relationships: is a type of pronucleus [GO:0045120] Sources: GOC:hjd, ISBN:0198506732 Definition: The pronucleus originating from the ovum that is being fertilized.